interferon regulatory factor 3-interferon regulatory factor 5 complex [GO:0097085] (cellular component) Also known as: IRF3:IRF5 complex Definition: An interferon regulatory factor complex that consists of a heterodimer of interferon regulatory factor 3 and interferon regulatory factor 5. Relationships: is a type of GO:0097071 References: PMID:12138184 Sources: GOC:cna